type II site-specific deoxyribonuclease complex [GO:0009359] (cellular component) Also known as: type II restriction enzyme complex Relationships: is a type of endodeoxyribonuclease complex [GO:1905347]; is part of cytoplasm [GO:0005737] References: PMID:12654995 Definition: A protein complex that functions as an endonuclease to cleave DNA at or near a specific recognition site, when that site is unmethylated. These complexes may be dimers or tetramers; it is also possible for the endonuclease to be in a complex with the corresponding methyltransferase that methylates the recognition site. DNA restriction systems such as this are used by bacteria to defend against phage and other foreign DNA that may enter a cell.